trichocyst [GO:0055039] (cellular component) Relationships: is a type of extracellular membraneless organelle [GO:0043264] Definition: A crystalline exocytotic organelle composed of small, acidic proteins existing primarily as disulphide-linked dimers. The trichocyst is an organelle that releases long filamentous proteins that capture predators in net-like structures, to slow them down when the cell is disturbed. The protein is nontoxic and shaped like a long, striated, fibrous shaft. References: PMID:3667715 Sources: GOC:jid, GOC:rph